positive regulation of xanthone-containing compound biosynthetic process [GO:1900185] (biological process) Definition: Any process that activates or increases the frequency, rate or extent of xanthone-containing compound biosynthetic process. Sources: GOC:TermGenie, GOC:di Also known as: activation of xanthone-containing compound anabolism, activation of xanthone-containing compound biosynthesis, activation of xanthone-containing compound formation, activation of xanthone-containing compound synthesis, positive regulation of xanthone-containing compound anabolism, positive regulation of xanthone-containing compound biosynthesis, positive regulation of xanthone-containing compound formation, positive regulation of xanthone-containing compound synthesis, up regulation of xanthone-containing compound anabolism, up regulation of xanthone-containing compound biosynthesis, up regulation of xanthone-containing compound biosynthetic process, up regulation of xanthone-containing compound formation, up regulation of xanthone-containing compound synthesis, up-regulation of xanthone-containing compound anabolism, up-regulation of xanthone-containing compound biosynthesis, up-regulation of xanthone-containing compound biosynthetic process, up-regulation of xanthone-containing compound formation, up-regulation of xanthone-containing compound synthesis, upregulation of xanthone-containing compound anabolism, upregulation of xanthone-containing compound biosynthesis, upregulation of xanthone-containing compound biosynthetic process, upregulation of xanthone-containing compound formation, upregulation of xanthone-containing compound synthesis, activation of xanthone biosynthesis, activation of xanthone biosynthetic process, activation of xanthone-containing compound biosynthetic process, positive regulation of xanthone biosynthesis, positive regulation of xanthone biosynthetic process, up regulation of xanthone biosynthesis, up regulation of xanthone biosynthetic process, up-regulation of xanthone biosynthesis, up-regulation of xanthone biosynthetic process, upregulation of xanthone biosynthesis, upregulation of xanthone biosynthetic process Relationships: is a type of positive regulation of biosynthetic process [GO:0009891]; is_a GO:0062013; is a type of GO:1900183; positively regulates GO:2001307 Subtypes: positive regulation of emericellin biosynthetic process [GO:1900836]